indole-3-carbonyl nitrile 4-hydroxylase activity [GO:0106149] (molecular function) References: PMID:26352477 Sources: GOC:lr, RHEA:57864 Definition: Catalysis of the reaction: indole-3-carbonyl nitrile + NADPH +O2=4-hydroxyindole-3- carbonyl nitrile + NADP+ + H20. Relationships: is a type of oxidoreductase activity, acting on paired donors, with incorporation or reduction of molecular oxygen, NAD(P)H as one donor, and incorporation of one atom of oxygen [GO:0016709]